{
  "gene_symbol": "TIMM29",
  "gene_name": "Mitochondrial import inner membrane translocase subunit Tim29",
  "gene": "UniProtKB:Q9BSF4",
  "term_id": "UNKNOWN:0001",
  "term_label": "Unknown molecular function"
}